male courtship behavior, orientation prior to leg tapping and wing vibration [GO:0016543] (biological process) Relationships: is a type of male courtship behavior [GO:0008049] Also known as: male courtship behavior, orientation, male courtship behaviour, orientation, male courtship behaviour, orientation prior to leg tapping and wing vibration References: PMID:11092827 Sources: GOC:sensu Definition: The process during courtship, where the male orients towards a potential partner. An example of this is found in Drosophila melanogaster.